{
  "term_id": "GO:0070507",
  "gene": "UniProtKB:Q9H9H5",
  "gene_name": "MAP6 domain-containing protein 1",
  "gene_symbol": "MAP6D1",
  "term_label": "regulation of microtubule cytoskeleton organization"
}